(hydroxyamino)benzene mutase activity [GO:0018824] (molecular function) Definition: Catalysis of the reaction: (hydroxyamino)benzene = 2-aminophenol. Relationships: is a type of intramolecular hydroxytransferase activity [GO:0050486] Also known as: (hydroxyamino)benzene hydroxymutase activity, HAB mutase activity, hydroxylaminobenzene hydroxymutase activity, hydroxylaminobenzene mutase activity Sources: EC:5.4.4.1, UM-BBD_reactionID:r0304